{
  "term_id": "GO:0031625",
  "gene_symbol": "SNCAIP",
  "gene": "UniProtKB:Q9Y6H5",
  "term_label": "ubiquitin protein ligase binding",
  "gene_name": "Synphilin-1"
}